9-cis-beta-carotene 9',10'-cleavage oxygenase activity [GO:0102395] (molecular function) Definition: Catalysis of the reaction: 9-cis-beta-carotene + O2 = 9-cis-10'-apo-beta-carotenal + beta-ionone. Relationships: is a type of oxidoreductase activity, acting on single donors with incorporation of molecular oxygen, incorporation of two atoms of oxygen [GO:0016702] Sources: EC:1.13.11.68, GOC:pz